{
  "gene_name": "E3 ubiquitin-protein ligase DTX3L",
  "gene_symbol": "DTX3L",
  "term_label": "Notch signaling pathway",
  "term_id": "GO:0007219",
  "gene": "UniProtKB:Q8TDB6"
}